ligand-modulated transcription activator activity [GO:0141097] (molecular function) Definition: A DNA-binding transcription activator activity regulated by binding to a ligand and that activates the transcription of specific genes and gene sets. Relationships: is a type of GO:0001216; is a type of ligand-modulated transcription factor activity [GO:0098531] Sources: GOC:pg Also known as: ligand-activated transcription activator activity